protein transport to mating projection actin fusion focus [GO:1904601] (biological process) Relationships: is a type of GO:0015031 References: PMID:25825517 Sources: GOC:TermGenie, GO_REF:0000087 Also known as: protein localisation in actin fusion focus, protein localisation to actin fusion focus, protein localization in actin fusion focus Definition: A process in which a protein is transported to a location within an actin fusion focus.